{
  "term_id": "UNKNOWN:0002",
  "gene_symbol": "OR51B2",
  "gene_name": "Olfactory receptor 51B2",
  "term_label": "Unknown biological process",
  "gene": "UniProtKB:Q9Y5P1"
}